{
  "term_id": "GO:0004143",
  "gene": "UniProtKB:O75912",
  "gene_symbol": "DGKI",
  "term_label": "ATP-dependent diacylglycerol kinase activity",
  "gene_name": "Diacylglycerol kinase iota"
}